{
  "gene_symbol": "EBF3",
  "term_label": "regulation of transcription by RNA polymerase II",
  "gene": "UniProtKB:Q9H4W6",
  "term_id": "GO:0006357",
  "gene_name": "Transcription factor COE3"
}